peroxidase-heme linkage [GO:0018186] (biological process) Also known as: peroxidase-haem linkage Relationships: is_a protein-heme linkage [GO:0017003]; is a type of cytochrome complex assembly [GO:0017004] Definition: The covalent linkage of heme to peroxidase. Sources: RESID:AA0279, RESID:AA0280